{
  "gene": "UniProtKB:Q7LBC6",
  "gene_name": "Lysine-specific demethylase 3B",
  "term_id": "GO:0031490",
  "gene_symbol": "KDM3B",
  "term_label": "chromatin DNA binding"
}